{
  "term_id": "GO:0005634",
  "gene": "UniProtKB:P31268",
  "gene_symbol": "HOXA7",
  "gene_name": "Homeobox protein Hox-A7",
  "term_label": "nucleus"
}